positive regulation of cartilage development [GO:0061036] (biological process) Definition: Any process that increases the rate, frequency, or extent of cartilage development, the process whose specific outcome is the progression of the cartilage over time, from its formation to the mature structure. Cartilage is a connective tissue dominated by extracellular matrix containing collagen type II and large amounts of proteoglycan, particularly chondroitin sulfate. Sources: GOC:dph Relationships: is a type of positive regulation of developmental process [GO:0051094]; is a type of positive regulation of multicellular organismal process [GO:0051240]; is a type of GO:0061035; positively regulates cartilage development [GO:0051216] Subtypes: positive regulation of chondrocyte differentiation [GO:0032332]